{
  "term_label": "Unknown molecular function",
  "gene_symbol": "PHF20L1",
  "term_id": "UNKNOWN:0001",
  "gene_name": "PHD finger protein 20-like protein 1",
  "gene": "UniProtKB:A8MW92"
}